{
  "gene": "UniProtKB:Q9Y2D4",
  "gene_symbol": "EXOC6B",
  "term_id": "GO:0006887",
  "term_label": "exocytosis",
  "gene_name": "Exocyst complex component 6B"
}